varicosity [GO:0043196] (cellular component) Definition: Non-terminal inflated portion of the axon, containing the specialized apparatus necessary to release neurotransmitters. Relationships: is a type of cellular anatomical structure [GO:0110165]; is part of main axon [GO:0044304] Sources: GOC:nln